{
  "gene": "UniProtKB:Q9H2A2",
  "term_label": "retinoic acid metabolic process",
  "gene_name": "2-aminomuconic semialdehyde dehydrogenase",
  "gene_symbol": "ALDH8A1",
  "term_id": "GO:0042573"
}